{
  "gene_name": "Glucose-6-phosphate exchanger SLC37A1",
  "term_id": "GO:0061513",
  "term_label": "glucose 6-phosphate:phosphate antiporter activity",
  "gene": "UniProtKB:P57057",
  "gene_symbol": "SLC37A1"
}